DNA-mediated transformation [GO:0009294] (biological process) Relationships: is a type of horizontal gene transfer [GO:0009292] Also known as: DNA mediated transformation References: PMID:12706993, PMID:24509783, PMID:27826682 Definition: The direct uptake and incorporation of exogenous genetic material (DNA or RNA) into a cell from its surroundings through the cell envelope.